{
  "gene_name": "Interleukin-23 subunit alpha",
  "gene": "UniProtKB:Q9NPF7",
  "term_id": "GO:0042102",
  "gene_symbol": "IL23A",
  "term_label": "positive regulation of T cell proliferation"
}